{
  "term_label": "chromosome condensation",
  "gene_name": "Histone H1.4",
  "term_id": "GO:0030261",
  "gene_symbol": "H1-4",
  "gene": "UniProtKB:P10412"
}